3-oxo-5-alpha-steroid 4-dehydrogenase activity [GO:0003865] (molecular function) Definition: Catalysis of the reaction: a 3-oxo-5-alpha-steroid + acceptor = a 3-oxo-delta(4)-steroid + reduced acceptor. Sources: EC:1.3.99.5 Also known as: 3-oxosteroid delta4-dehydrogenase, 5alpha-reductase, delta4-3-oxosteroid-5alpha-reductase, steroid 5 alpha reductase, steroid 5-alpha-reductase activity, steroid 5alpha-reductase, testosterone 5alpha-reductase, 3-keto-delta4-steroid-5alpha-reductase activity, 3-oxo-5alpha-steroid 4-dehydrogenase activity, 3-oxo-5alpha-steroid delta4-dehydrogenase activity, 3-oxo-5alpha-steroid:(acceptor) delta4-oxidoreductase activity, 3-oxo-5alpha-steroid:acceptor delta4-oxidoreductase activity, 4-ene-3-ketosteroid-5alpha-oxidoreductase activity, delta4-3-keto steroid 5alpha-reductase activity, delta4-3-ketosteroid5alpha-oxidoreductase activity, delta4-3-oxo steroid reductase activity, delta4-5alpha-dehydrogenase activity, steroid delta4-5alpha-reductase activity Relationships: is a type of GO:0033765 Subtypes: 3-oxo-5-alpha-steroid 4-dehydrogenase (NADP+) activity [GO:0047751]